sideretin biosynthesis [GO:0106146] (biological process) References: PMID:29581584 Sources: GOC:lr Definition: The chemical reactions and pathways resulting in the formation of sideretin. Relationships: is a type of coumarin biosynthetic process [GO:0009805]